{
  "gene": "UniProtKB:Q9NPR2",
  "term_id": "GO:0001755",
  "term_label": "neural crest cell migration",
  "gene_name": "Semaphorin-4B",
  "gene_symbol": "SEMA4B"
}